regulation of primitive erythrocyte differentiation [GO:0010725] (BP) Definition: Any process that modulates the rate, frequency, or extent of primitive erythrocyte differentiation. Primitive erythrocyte differentiation occurs as part of the process of primitive hemopoiesis. Relationships: is a type of regulation of erythrocyte differentiation [GO:0045646]; regulates primitive erythrocyte differentiation [GO:0060319] Sources: GOC:add, GOC:dph, GOC:tb Also known as: regulation of primitive RBC differentiation, regulation of primitive erythropoeisis, regulation of primitive red blood cell differentiation